{
  "gene": "UniProtKB:Q9BZJ8",
  "gene_symbol": "GPR61",
  "term_label": "endosome",
  "gene_name": "G-protein coupled receptor 61",
  "term_id": "GO:0005768"
}